pollen-style interaction [GO:0140302] (biological process) References: PMID:27899537 Definition: The interactions (or cell to cell communication) that occur between the male gametophyte (pollen/pollen tube) and the stylar tissues of the female sporophyte. Relationships: is a type of pollen-pistil interaction [GO:0009875]